{
  "term_id": "GO:0005654",
  "gene_symbol": "EID1",
  "gene": "UniProtKB:Q9Y6B2",
  "term_label": "nucleoplasm",
  "gene_name": "EP300-interacting inhibitor of differentiation 1"
}